pronephric nephron tubule formation [GO:0039006] (biological process) Also known as: pronephric tubule formation, pronephros tubule formation Sources: GOC:mtg_kidney_jan10 Definition: The developmental process pertaining to the initial formation of a pronephric nephron tubule from unspecified parts. A pronephric nephron tubule is an epithelial tube that is part of a nephron in the pronephros. Relationships: is a type of GO:0072079; is part of pronephric nephron tubule morphogenesis [GO:0039008]; is part of pronephros formation [GO:0072116]